{
  "term_id": "GO:0009897",
  "gene_symbol": "FCGR3A",
  "term_label": "external side of plasma membrane",
  "gene": "UniProtKB:P08637",
  "gene_name": "Low affinity immunoglobulin gamma Fc region receptor III-A"
}